{
  "gene_name": "tRNA 2'-phosphotransferase 1",
  "term_label": "tRNA 2'-phosphotransferase activity",
  "gene": "UniProtKB:Q86TN4",
  "term_id": "GO:0000215",
  "gene_symbol": "TRPT1"
}